{
  "gene": "UniProtKB:P28223",
  "term_id": "GO:0007208",
  "term_label": "phospholipase C-activating serotonin receptor signaling pathway",
  "gene_name": "5-hydroxytryptamine receptor 2A",
  "gene_symbol": "HTR2A"
}